{
  "gene": "UniProtKB:Q16621",
  "term_id": "GO:0006357",
  "gene_name": "Transcription factor NF-E2 45 kDa subunit",
  "gene_symbol": "NFE2",
  "term_label": "regulation of transcription by RNA polymerase II"
}